{
  "gene_name": "Transcription factor 24",
  "term_id": "GO:0000977",
  "gene_symbol": "TCF24",
  "term_label": "RNA polymerase II transcription regulatory region sequence-specific DNA binding",
  "gene": "UniProtKB:Q7RTU0"
}